{
  "gene_name": "Protein CBFA2T2",
  "term_id": "GO:0005634",
  "gene_symbol": "CBFA2T2",
  "gene": "UniProtKB:O43439",
  "term_label": "nucleus"
}